positive regulation of toll-like receptor 10 signaling pathway [GO:0034169] (biological process) References: PMID:16551253, PMID:17328678 Sources: GOC:add Relationships: is a type of regulation of toll-like receptor 10 signaling pathway [GO:0034167]; is a type of positive regulation of pattern recognition receptor signaling pathway [GO:0062208]; positively regulates toll-like receptor 10 signaling pathway [GO:0034166] Also known as: positive regulation of TLR10 signaling pathway, positive regulation of toll-like receptor 10 signalling pathway Definition: Any process that activates or increases the frequency, rate, or extent of toll-like receptor 10 signaling pathway.